{
  "gene": "UniProtKB:B2RC85",
  "gene_name": "Radial spoke head 10 homolog B2",
  "term_id": "UNKNOWN:0001",
  "gene_symbol": "RSPH10B2",
  "term_label": "Unknown molecular function"
}